{
  "term_label": "axoneme",
  "term_id": "GO:0005930",
  "gene_symbol": "RSPH9",
  "gene_name": "Radial spoke head protein 9 homolog",
  "gene": "UniProtKB:Q9H1X1"
}